{
  "term_label": "endoplasmic reticulum",
  "term_id": "GO:0005783",
  "gene": "UniProtKB:O95994",
  "gene_name": "Anterior gradient protein 2 homolog",
  "gene_symbol": "AGR2"
}